{
  "gene_symbol": "RELCH",
  "gene": "UniProtKB:Q9P260",
  "term_id": "GO:0032367",
  "term_label": "intracellular cholesterol transport",
  "gene_name": "RAB11-binding protein RELCH"
}